argininosuccinate synthase activity [GO:0004055] (molecular function) Definition: Catalysis of the reaction: ATP + L-citrulline + L-aspartate = AMP + diphosphate + (N(omega)-L-arginino)succinate. Also known as: L-citrulline:L-aspartate ligase (AMP-forming), arginine succinate synthetase activity, argininosuccinate synthetase activity, argininosuccinic acid synthetase activity, arginosuccinate synthetase activity, citrulline--aspartate ligase activity Relationships: is a type of GO:0016879 Sources: EC:6.3.4.5